4,5-dihydroxyphthalate decarboxylase activity [GO:0018796] (molecular function) Relationships: is a type of GO:0016831 Also known as: 4,5-dihydroxyphthalate carboxy-lyase (3,4-dihydroxybenzoate-forming), 4,5-dihydroxyphthalate carboxy-lyase activity Definition: Catalysis of the reaction: 4,5-dihydroxyphthalate = 3,4-dihydroxybenzoate + CO2. Sources: EC:4.1.1.55